{
  "term_id": "GO:0005737",
  "gene": "UniProtKB:P0DMV8",
  "term_label": "cytoplasm",
  "gene_name": "Heat shock 70 kDa protein 1A",
  "gene_symbol": "HSPA1A"
}